{
  "term_label": "cell fate commitment",
  "gene": "UniProtKB:Q9BWX5",
  "gene_symbol": "GATA5",
  "gene_name": "Transcription factor GATA-5",
  "term_id": "GO:0045165"
}